{
  "term_id": "GO:0061630",
  "term_label": "ubiquitin protein ligase activity",
  "gene_name": "E3 ubiquitin-protein ligase RING2",
  "gene_symbol": "RNF2",
  "gene": "UniProtKB:Q99496"
}